{
  "term_label": "transmembrane transport",
  "gene": "UniProtKB:P04920",
  "term_id": "GO:0055085",
  "gene_symbol": "SLC4A2",
  "gene_name": "Anion exchange protein 2"
}